{
  "gene_symbol": "PADI2",
  "gene": "UniProtKB:Q9Y2J8",
  "term_id": "GO:0006338",
  "term_label": "chromatin remodeling",
  "gene_name": "Protein-arginine deiminase type-2"
}